snRNA transport [GO:0051030] (biological process) Definition: The directed movement of snRNA, small nuclear ribonucleic acid, into, out of or within a cell, or between cells, by means of some agent such as a transporter or pore. Relationships: is a type of GO:0050658 Subtypes: snRNA export from nucleus [GO:0006408], GO:0061015 Sources: GOC:ai